{
  "term_label": "regulation of cytoplasmic translation",
  "gene_name": "Zinc finger protein 385A",
  "gene": "UniProtKB:Q96PM9",
  "gene_symbol": "ZNF385A",
  "term_id": "GO:2000765"
}